{
  "gene": "UniProtKB:P14324",
  "gene_name": "Farnesyl pyrophosphate synthase",
  "term_id": "GO:0004161",
  "gene_symbol": "FDPS",
  "term_label": "dimethylallyltranstransferase activity"
}